{
  "gene_symbol": "RPA1",
  "gene": "UniProtKB:P27694",
  "gene_name": "Replication protein A 70 kDa DNA-binding subunit",
  "term_label": "double-strand break repair via homologous recombination",
  "term_id": "GO:0000724"
}